{
  "term_id": "GO:0070776",
  "gene_symbol": "BRPF3",
  "term_label": "MOZ/MORF histone acetyltransferase complex",
  "gene": "UniProtKB:Q9ULD4",
  "gene_name": "Bromodomain and PHD finger-containing protein 3"
}